xanthoxin dehydrogenase (NAD+) activity [GO:0010301] (molecular function) Definition: Catalysis of the reaction: NAD+ + xanthoxin = (+)-abscisic aldehyde + H+ + NADH. Sources: EC:1.1.1.288, RHEA:12548 Also known as: xanthoxin dehydrogenase activity, ABA2, xanthoxin oxidase activity, xanthoxin:NAD+ oxidoreductase activity Relationships: is a type of GO:0004022